{
  "term_label": "mitochondrial small ribosomal subunit",
  "term_id": "GO:0005763",
  "gene_symbol": "MRPS22",
  "gene_name": "Small ribosomal subunit protein mS22",
  "gene": "UniProtKB:P82650"
}